{
  "gene_name": "Myosin-7B",
  "term_label": "myosin filament",
  "term_id": "GO:0032982",
  "gene": "UniProtKB:A7E2Y1",
  "gene_symbol": "MYH7B"
}